{
  "gene": "UniProtKB:Q5XG92",
  "gene_symbol": "CES4A",
  "term_id": "UNKNOWN:0002",
  "gene_name": "Carboxylesterase 4A",
  "term_label": "Unknown biological process"
}